matrilin complex [GO:0120216] (cellular component) Also known as: matrilin-1 complex, matrilin-2 complex, matrilin-3 complex, matrilin-4 complex, matrilin family complex References: PMID:10367731, PMID:15075323, PMID:9699631 Sources: GOC:bhm Definition: A cartilage extracellular matrix complex that mediates interactions between major components of the extracellular matrix such as collagens and proteoglycans and contributes to their fibrillar network. Exists as an obligate homotrimer. Relationships: is a type of protein-containing complex [GO:0032991]; is part of GO:0031012